{
  "term_id": "GO:0140410",
  "gene_name": "Zinc transporter ZIP4",
  "gene_symbol": "SLC39A4",
  "gene": "UniProtKB:Q6P5W5",
  "term_label": "monoatomic cation:bicarbonate symporter activity"
}